positive regulation of xyloglucan catabolic process [GO:2000953] (biological process) Also known as: positive regulation of xyloglucan catabolism Definition: Any process that activates or increases the frequency, rate or extent of xyloglucan catabolic process. Relationships: is a type of regulation of xyloglucan catabolic process [GO:2000951]; is a type of GO:2000990; positively regulates GO:2000899 Sources: GOC:mengo_curators